{
  "term_id": "GO:0036064",
  "gene_symbol": "TTLL6",
  "gene": "UniProtKB:Q8N841",
  "term_label": "ciliary basal body",
  "gene_name": "Tubulin polyglutamylase TTLL6"
}